{
  "gene_symbol": "C6orf50",
  "gene": "UniProtKB:Q9HD87",
  "term_id": "UNKNOWN:0001",
  "gene_name": "Putative uncharacterized protein C6orf50",
  "term_label": "Unknown molecular function"
}